{
  "gene_symbol": "NIPSNAP3A",
  "term_id": "UNKNOWN:0002",
  "term_label": "Unknown biological process",
  "gene": "UniProtKB:Q9UFN0",
  "gene_name": "Protein NipSnap homolog 3A"
}